{
  "term_id": "GO:0008375",
  "gene": "UniProtKB:Q9UBM8",
  "term_label": "acetylglucosaminyltransferase activity",
  "gene_symbol": "MGAT4C",
  "gene_name": "Alpha-1,3-mannosyl-glycoprotein 4-beta-N-acetylglucosaminyltransferase C"
}